{
  "term_id": "UNKNOWN:0001",
  "gene_symbol": "TRAV16",
  "gene": "UniProtKB:A0A0A6YYK6",
  "term_label": "Unknown molecular function",
  "gene_name": "T cell receptor alpha variable 16"
}